{
  "gene_symbol": "FAM237B",
  "gene": "UniProtKB:A0A1B0GVD1",
  "term_id": "UNKNOWN:0002",
  "gene_name": "Protein FAM237B",
  "term_label": "Unknown biological process"
}